{
  "term_label": "plasma membrane",
  "gene": "UniProtKB:Q14156",
  "gene_symbol": "EFR3A",
  "term_id": "GO:0005886",
  "gene_name": "Protein EFR3 homolog A"
}